{
  "term_id": "GO:0005634",
  "gene": "UniProtKB:P28065",
  "term_label": "nucleus",
  "gene_symbol": "PSMB9",
  "gene_name": "Proteasome subunit beta type-9"
}